{
  "term_id": "GO:0007268",
  "gene_name": "Proenkephalin-B",
  "gene": "UniProtKB:P01213",
  "term_label": "chemical synaptic transmission",
  "gene_symbol": "PDYN"
}